{
  "gene_symbol": "PSMD7",
  "term_id": "GO:0000502",
  "gene_name": "26S proteasome non-ATPase regulatory subunit 7",
  "term_label": "proteasome complex",
  "gene": "UniProtKB:P51665"
}